primary sex determination, soma [GO:0007539] (biological process) Sources: GOC:ems Relationships: is a type of primary sex determination [GO:0007538]; is part of somatic sex determination [GO:0018993] Definition: The transmission of information about sexual status from the initial, general, determination to signals specific to the soma.